formimidoylaspartate deiminase activity [GO:0050414] (molecular function) Also known as: formiminoaspartate deiminase activity, N-formimidoyl-L-aspartate iminohydrolase activity Definition: Catalysis of the reaction: N-formimidoyl-L-aspartate + H2O = N-formyl-L-aspartate + NH3. Relationships: is a type of hydrolase activity, acting on carbon-nitrogen (but not peptide) bonds, in linear amidines [GO:0016813] Sources: EC:3.5.3.5, MetaCyc:FORMIMINOASPARTATE-DEIMINASE-RXN